spermidine:sinapoyl CoA N-acyltransferase activity [GO:0080072] (molecular function) Definition: Catalysis of the transfer of a sinapoyl group to a nitrogen atom on the spermidine molecule. References: PMID:19077165 Relationships: is a type of GO:0016410